{
  "gene_symbol": "TTLL7",
  "gene_name": "Tubulin polyglutamylase TTLL7",
  "term_label": "tubulin-glutamic acid ligase activity",
  "term_id": "GO:0070740",
  "gene": "UniProtKB:Q6ZT98"
}